{
  "term_id": "GO:0050291",
  "gene_symbol": "CERS1",
  "term_label": "sphingosine N-acyltransferase activity",
  "gene_name": "Ceramide synthase 1",
  "gene": "UniProtKB:P27544"
}